{
  "term_label": "protein serine/threonine kinase activity",
  "gene_name": "Serine_threonine-protein kinase ULK3",
  "gene": "UniProtKB:Q6PHR2",
  "term_id": "GO:0004674",
  "gene_symbol": "ULK3"
}